double-strand break repair [GO:0006302] (biological process) Relationships: is a type of DNA repair [GO:0006281] Sources: GOC:elh Note: Note that the processes of nuclear double-strand break repair and mitochondrial double-strand break repair are genetically separable (PMID:22214610). To annotate gene products involved in mitochondrial double-strand break repair, please use GO:0097551 'mitochondrial double-strand break repair'. Regulation: RO_0002211 by GO:2000779; negatively regulated by negative regulation of double-strand break repair [GO:2000780]; positively regulated by GO:2000781 Definition: The repair of double-strand breaks in DNA via homologous and nonhomologous mechanisms to reform a continuous DNA helix. Subtypes: GO:0000724, double-strand break repair via nonhomologous end joining [GO:0006303], double-strand break repair via single-strand annealing [GO:0045002], GO:0097551, GO:1990918